T-bar [GO:0098986] (cellular component) Definition: A T-shaped presynpatic density. These are common in arhropod central nervous systems. References: PMID:26780543 Sources: GOC:dos Relationships: is a type of presynaptic density [GO:0098980]